vesicle fusion [GO:0006906] (biological process) Regulation: regulated by regulation of vesicle fusion [GO:0031338]; negatively regulated by negative regulation of vesicle fusion [GO:0031339]; positively regulated by GO:0031340 Relationships: is a type of vesicle organization [GO:0016050]; is a type of organelle membrane fusion [GO:0090174]; is part of GO:0016192 Definition: Fusion of the membrane of a transport vesicle with its target membrane. Sources: GOC:jid Subtypes: vesicle fusion with nuclear membrane involved in mitotic nuclear envelope reassembly [GO:0007086], vesicle fusion with peroxisome [GO:0019817], GO:0034058, Golgi vesicle fusion to target membrane [GO:0048210], GO:0048279, GO:0048280, vesicle fusion with vacuole [GO:0051469], multivesicular body-lysosome fusion [GO:0061763], vesicle fusion with vesicle [GO:0061782], autophagosome-lysosome fusion [GO:0061909], GO:0061910, amphisome-lysosome fusion [GO:0061911], phagosome-lysosome fusion [GO:0090385], vesicle fusion to plasma membrane [GO:0099500], proacrosomal vesicle fusion [GO:0120211], GO:0160156, vesicle fusion with endoplasmic reticulum-Golgi intermediate compartment (ERGIC) membrane [GO:1990668], GO:1990670